positive regulation of glycoprotein biosynthetic process [GO:0010560] (biological process) Subtypes: positive regulation of amyloid precursor protein biosynthetic process [GO:0042986], positive regulation of proteoglycan biosynthetic process [GO:1902730], GO:1904100, positive regulation of glycoprotein biosynthetic process involved in immunological synapse formation [GO:2000526] Definition: Any process that increases the rate, frequency, or extent of the chemical reactions and pathways resulting in the formation of a glycoprotein, a protein that contains covalently bound glycose (i.e. monosaccharide) residues; the glycose occurs most commonly as oligosaccharide or fairly small polysaccharide but occasionally as monosaccharide. Sources: GOC:dph, GOC:tb Relationships: is a type of positive regulation of macromolecule biosynthetic process [GO:0010557]; is a type of GO:0010559; is a type of positive regulation of glycoprotein metabolic process [GO:1903020]; positively regulates glycoprotein biosynthetic process [GO:0009101]